sugar mediated signaling pathway [GO:0010182] (biological process) Subtypes: GO:0009745, hexose mediated signaling [GO:0009757] References: PMID:9014361 Also known as: sugar mediated signalling Definition: The process in which a change in the level of a mono- or disaccharide such as glucose, fructose or sucrose triggers the expression of genes controlling metabolic and developmental processes. Relationships: is_a carbohydrate mediated signaling [GO:0009756]